{
  "term_label": "long-term synaptic potentiation",
  "term_id": "GO:0060291",
  "gene_symbol": "GRIN2D",
  "gene_name": "Glutamate receptor ionotropic, NMDA 2D",
  "gene": "UniProtKB:O15399"
}